negative regulation of methane biosynthetic process from dimethyl sulfide [GO:1900343] (BP) Definition: Any process that stops, prevents or reduces the frequency, rate or extent of methane biosynthetic process from dimethyl sulfide. Sources: GOC:TermGenie, GOC:mengo_curators Also known as: down regulation of methane biosynthetic process from dimethyl sulfide, down-regulation of methane biosynthetic process from dimethyl sulfide, downregulation of methane biosynthetic process from dimethyl sulfide, inhibition of methane biosynthetic process from dimethyl sulfide Relationships: is a type of GO:1900342; is a type of negative regulation of alkane biosynthetic process [GO:1901578]; is a type of GO:1901856; negatively regulates methane biosynthetic process from dimethyl sulfide [GO:2001131]